{
  "gene_symbol": "TRO",
  "gene_name": "Trophinin",
  "gene": "UniProtKB:Q12816",
  "term_id": "GO:0000122",
  "term_label": "negative regulation of transcription by RNA polymerase II"
}